{
  "term_id": "GO:0000981",
  "gene_symbol": "HOXA11",
  "term_label": "DNA-binding transcription factor activity, RNA polymerase II-specific",
  "gene": "UniProtKB:P31270",
  "gene_name": "Homeobox protein Hox-A11"
}